catalytic activity, acting on RNA [GO:0140098] (MF) Subtypes: first spliceosomal transesterification activity [GO:0000384], second spliceosomal transesterification activity [GO:0000386], RNA helicase activity [GO:0003724], RNA-3'-phosphate cyclase activity [GO:0003963], RNA nuclease activity [GO:0004540], RNA methyltransferase activity [GO:0008173], RNA guanylyltransferase activity [GO:0008192], RNA ligase activity [GO:0008452], RNA glycosylase activity [GO:0030597], GO:0033592, DNA/RNA helicase activity [GO:0033677], mRNA 5'-diphosphatase activity [GO:0034353], GO:0035515, tyrosyl-RNA phosphodiesterase activity [GO:0036317], GO:0050265, RNA polymerase activity [GO:0097747], template-free RNA nucleotidyltransferase [GO:0098680], snRNA pseudouridine synthase activity [GO:0106032], RNA NAD+-cap (NAD+-forming) hydrolase activity [GO:0110152], GO:0110153, rRNA pseudouridine synthase activity [GO:0120159], catalytic activity, acting on a tRNA [GO:0140101], catalytic activity, acting on a rRNA [GO:0140102], RNA topoisomerase activity [GO:0140226], mRNA 5'-triphosphate monophosphatase activity [GO:0140818], RNA 2',3'-cyclic phosphatase activity [GO:0160272], RNA 2'-phosphatase activity [GO:0160273] Definition: Catalytic activity that acts to modify RNA. Sources: GOC:molecular_function_refactoring, GOC:pdt Relationships: is a type of catalytic activity, acting on a nucleic acid [GO:0140640]